{
  "term_label": "positive regulation of fat cell differentiation",
  "gene": "UniProtKB:Q9H7C9",
  "gene_symbol": "AAMDC",
  "gene_name": "Mth938 domain-containing protein",
  "term_id": "GO:0045600"
}